{
  "term_id": "GO:0010468",
  "gene_symbol": "TRIM77",
  "gene": "UniProtKB:I1YAP6",
  "gene_name": "Tripartite motif-containing protein 77",
  "term_label": "regulation of gene expression"
}